{
  "gene": "UniProtKB:P46089",
  "term_label": "adenylate cyclase-activating G protein-coupled receptor signaling pathway",
  "gene_symbol": "GPR3",
  "gene_name": "G-protein coupled receptor 3",
  "term_id": "GO:0007189"
}